{
  "gene_symbol": "PNPLA5",
  "gene": "UniProtKB:Q7Z6Z6",
  "term_id": "GO:0016020",
  "gene_name": "Patatin-like phospholipase domain-containing protein 5",
  "term_label": "membrane"
}